{
  "gene_name": "TP53-regulated inhibitor of apoptosis 1",
  "term_label": "phosphatidic acid transfer activity",
  "gene_symbol": "TRIAP1",
  "gene": "UniProtKB:O43715",
  "term_id": "GO:1990050"
}